{
  "gene_symbol": "CLPSL2",
  "term_label": "enzyme activator activity",
  "gene": "UniProtKB:Q6UWE3",
  "gene_name": "Colipase-like protein 2",
  "term_id": "GO:0008047"
}